purine deoxyribonucleotide binding [GO:0032554] (molecular function) Sources: GOC:mah Relationships: is a type of purine nucleotide binding [GO:0017076]; is a type of GO:0032552 Definition: Binding to a purine deoxyribonucleotide, any compound consisting of a purine deoxyribonucleoside that is esterified with (ortho)phosphate or an oligophosphate at any hydroxyl group on the deoxyribose moiety. Subtypes: adenyl deoxyribonucleotide binding [GO:0032558], guanyl deoxyribonucleotide binding [GO:0032560]